vesicle fusion with endoplasmic reticulum-Golgi intermediate compartment (ERGIC) membrane [GO:1990668] (biological process) Definition: The joining of the lipid bilayer membrane around a vesicle to the lipid bilayer membrane of the ERGIC. This can involve anterograde or retrograde transport vesicles. References: PMID:16038056, PMID:24119662 Sources: GOC:bhm Also known as: vesicle fusion with ER-Golgi intermediate compartment (ERGIC) membrane, vesicle fusion with ER-Golgi intermediate compartment membrane, vesicle fusion with ERGIC membrane, vesicle fusion with endoplasmic reticulum-Golgi intermediate compartment membrane Relationships: is a type of vesicle fusion [GO:0006906] Subtypes: endoplasmic reticulum-derived vesicle fusion with endoplasmic reticulum-Golgi intermediate compartment (ERGIC) membrane [GO:1990687], Golgi vesicle fusion with endoplasmic reticulum-Golgi intermediate compartment (ERGIC) membrane [GO:1990688]